{
  "gene": "UniProtKB:P05305",
  "term_label": "endothelin A receptor binding",
  "term_id": "GO:0031707",
  "gene_symbol": "EDN1",
  "gene_name": "Endothelin-1"
}